oligopeptide import across plasma membrane [GO:0140205] (biological process) Relationships: is a type of oligopeptide transmembrane transport [GO:0035672]; is a type of import across plasma membrane [GO:0098739] Subtypes: dipeptide import across plasma membrane [GO:0140206], GO:0140207, tetrapeptide import across plasma membrane [GO:1901583] Definition: The directed movement of an oligopeptide from outside of a cell, across the plasma membrane and into the cytosol. References: PMID:22226946